tRNA pseudouridine(38/39) synthase activity [GO:0160154] (molecular function) Definition: Catalysis of the reaction: uridine(38/39) in tRNA = pseudouridine(38/39) in tRNA. Relationships: is a type of tRNA pseudouridine synthase activity [GO:0106029] Sources: EC:5.4.99.45